{
  "gene_symbol": "NSMCE1",
  "term_id": "GO:0000724",
  "term_label": "double-strand break repair via homologous recombination",
  "gene_name": "Non-structural maintenance of chromosomes element 1 homolog",
  "gene": "UniProtKB:Q8WV22"
}